negative regulation of antigen processing and presentation of peptide antigen via MHC class II [GO:0002587] (biological process) Sources: GOC:add Definition: Any process that stops, prevents, or reduces the frequency, rate, or extent of antigen processing and presentation of peptide antigen via MHC class II. Relationships: is a type of negative regulation of antigen processing and presentation of peptide or polysaccharide antigen via MHC class II [GO:0002581]; is a type of negative regulation of antigen processing and presentation of peptide antigen [GO:0002584]; is a type of GO:0002586; negatively regulates antigen processing and presentation of peptide antigen via MHC class II [GO:0002495] Also known as: down regulation of antigen processing and presentation of peptide antigen via MHC class II, down-regulation of antigen processing and presentation of peptide antigen via MHC class II, downregulation of antigen processing and presentation of peptide antigen via MHC class II, negative regulation of peptide antigen processing and presentation via MHC class II, inhibition of antigen processing and presentation of peptide antigen via MHC class II